{
  "gene": "UniProtKB:Q9BX26",
  "term_label": "Unknown molecular function",
  "gene_name": "Synaptonemal complex protein 2",
  "gene_symbol": "SYCP2",
  "term_id": "UNKNOWN:0001"
}